positive regulation of acute inflammatory response [GO:0002675] (biological process) Relationships: is_a GO:0002673; is a type of GO:0050729; positively regulates acute inflammatory response [GO:0002526] Sources: GOC:add Also known as: up regulation of acute inflammatory response, up-regulation of acute inflammatory response, upregulation of acute inflammatory response, activation of acute inflammatory response, stimulation of acute inflammatory response Definition: Any process that activates or increases the frequency, rate, or extent of an acute inflammatory response. Subtypes: GO:0002258, positive regulation of acute inflammatory response to antigenic stimulus [GO:0002866], positive regulation of acute inflammatory response to non-antigenic stimulus [GO:0002879], GO:0031622